{
  "term_label": "plasma membrane",
  "gene_name": "Protocadherin alpha-10",
  "term_id": "GO:0005886",
  "gene_symbol": "PCDHA10",
  "gene": "UniProtKB:Q9Y5I2"
}